{
  "gene_name": "Cadherin-24",
  "gene": "UniProtKB:Q86UP0",
  "term_label": "cadherin binding",
  "gene_symbol": "CDH24",
  "term_id": "GO:0045296"
}